{
  "term_label": "structural constituent of eye lens",
  "term_id": "GO:0005212",
  "gene_symbol": "CRYGD",
  "gene": "UniProtKB:P07320",
  "gene_name": "Gamma-crystallin D"
}